{
  "term_id": "GO:0000146",
  "gene_symbol": "MYH2",
  "gene_name": "Myosin-2",
  "gene": "UniProtKB:Q9UKX2",
  "term_label": "microfilament motor activity"
}